{
  "gene_symbol": "ETV1",
  "term_label": "DNA-binding transcription factor activity, RNA polymerase II-specific",
  "gene_name": "ETS translocation variant 1",
  "gene": "UniProtKB:P50549",
  "term_id": "GO:0000981"
}